positive regulation of host-seeking behavior [GO:0032540] (biological process) Also known as: positive regulation of host-seeking behaviour, up regulation of host-seeking behavior, up-regulation of host-seeking behavior, upregulation of host-seeking behavior, activation of host-seeking behavior, stimulation of host-seeking behavior Definition: Any process that activates or increases the frequency, rate or extent of any behavior associated with finding a host organism. Relationships: is a type of regulation of host-seeking behavior [GO:0032538]; is a type of positive regulation of behavior [GO:0048520]; positively regulates host-seeking behavior [GO:0032537] Sources: GOC:mah